{
  "gene_name": "Peroxisomal N(1)-acetyl-spermine_spermidine oxidase",
  "gene_symbol": "PAOX",
  "gene": "UniProtKB:Q6QHF9",
  "term_label": "polyamine oxidase activity",
  "term_id": "GO:0046592"
}